{
  "gene_name": "Protein arginine N-methyltransferase 3",
  "gene": "UniProtKB:O60678",
  "term_label": "histone methyltransferase activity",
  "term_id": "GO:0042054",
  "gene_symbol": "PRMT3"
}